{
  "term_label": "intracellular protein localization",
  "term_id": "GO:0008104",
  "gene_symbol": "YWHAH",
  "gene": "UniProtKB:Q04917",
  "gene_name": "14-3-3 protein eta"
}